neuronal-glial interaction involved in cerebral cortex radial glia guided migration [GO:0021812] (biological process) Also known as: neuronal-glial interaction involved in cerebral cortex glial-mediated radial migration Definition: The changes in adhesion between neuronal cells and glial cells as a component of the process of cerebral cortex glial-mediated radial cell migration. References: PMID:12626695 Sources: GOC:cls, GOC:dgh, GOC:dph, GOC:jid, GO_REF:0000021 Relationships: is a type of cell-cell adhesion [GO:0098609]; is part of cerebral cortex radial glia-guided migration [GO:0021801]